{
  "gene_name": "Piezo-type mechanosensitive ion channel component 2",
  "term_id": "GO:0008381",
  "term_label": "mechanosensitive monoatomic ion channel activity",
  "gene_symbol": "PIEZO2",
  "gene": "UniProtKB:Q9H5I5"
}